{
  "term_label": "perinuclear region of cytoplasm",
  "gene": "UniProtKB:Q8IZ41",
  "term_id": "GO:0048471",
  "gene_symbol": "RASEF",
  "gene_name": "Ras and EF-hand domain-containing protein"
}